{
  "gene": "UniProtKB:Q9H2K2",
  "gene_name": "Poly [ADP-ribose] polymerase tankyrase-2",
  "gene_symbol": "TNKS2",
  "term_id": "GO:0070198",
  "term_label": "protein localization to chromosome, telomeric region"
}